regulation of protein polymerization [GO:0032271] (biological process) Also known as: regulation of protein polymerisation Subtypes: regulation of actin filament polymerization [GO:0030833], GO:0030839, regulation of microtubule polymerization [GO:0031113], negative regulation of protein polymerization [GO:0032272], positive regulation of protein polymerization [GO:0032273], regulation of free ubiquitin chain polymerization [GO:1904542] Relationships: is a type of regulation of protein-containing complex assembly [GO:0043254]; regulates protein polymerization [GO:0051258] Sources: GOC:mah Definition: Any process that modulates the frequency, rate or extent of the process of creating protein polymers.